{
  "term_id": "GO:0070006",
  "gene_name": "Thyrotropin-releasing hormone-degrading ectoenzyme",
  "gene": "UniProtKB:Q9UKU6",
  "gene_symbol": "TRHDE",
  "term_label": "metalloaminopeptidase activity"
}